anthocyanin-containing compound biosynthetic process [GO:0009718] (biological process) Relationships: is a type of GO:0009813; is a type of pigment biosynthetic process [GO:0046148]; is a type of anthocyanin-containing compound metabolic process [GO:0046283] Also known as: anthocyanin anabolism, anthocyanin biosynthesis, anthocyanin biosynthetic process, anthocyanin formation, anthocyanin synthesis Definition: The chemical reactions and pathways resulting in the formation of anthocyanins, any member of a group of intensely colored soluble glycosides of anthocyanidins. Regulation: regulated by GO:0031540; negatively regulated by negative regulation of anthocyanin biosynthetic process [GO:0031541]; positively regulated by GO:0031542 Sources: GOC:ai Subtypes: anthocyanin biosynthetic process involved in anthocyanin accumulation in response to UV light [GO:0043483]